{
  "gene_symbol": "RWDD1",
  "gene_name": "RWD domain-containing protein 1",
  "gene": "UniProtKB:Q9H446",
  "term_id": "UNKNOWN:0001",
  "term_label": "Unknown molecular function"
}